{
  "term_id": "GO:0003713",
  "term_label": "transcription coactivator activity",
  "gene_symbol": "DYRK1B",
  "gene_name": "Dual specificity tyrosine-phosphorylation-regulated kinase 1B",
  "gene": "UniProtKB:Q9Y463"
}